{
  "gene_symbol": "ZNF644",
  "gene": "UniProtKB:Q9H582",
  "term_label": "DNA-binding transcription factor activity, RNA polymerase II-specific",
  "gene_name": "Zinc finger protein 644",
  "term_id": "GO:0000981"
}